negative regulation of aggrephagy [GO:1905336] (biological process) Also known as: down regulation of aggrephagy, down-regulation of aggrephagy, downregulation of aggrephagy, inhibition of aggrephagy References: PMID:25686248 Sources: GOC:PARL, GOC:TermGenie, GOC:pad, GO_REF:0000058 Relationships: is a type of GO:0016242; is a type of regulation of aggrephagy [GO:1905335]; negatively regulates aggrephagy [GO:0035973] Definition: Any process that stops, prevents or reduces the frequency, rate or extent of aggrephagy.